{
  "term_label": "isopentenyl-diphosphate delta-isomerase activity",
  "gene": "UniProtKB:Q13907",
  "term_id": "GO:0004452",
  "gene_symbol": "IDI1",
  "gene_name": "Isopentenyl-diphosphate Delta-isomerase 1"
}